meiosis II nuclear membrane disassembly [GO:0051080] (biological process) Relationships: is a type of meiotic nuclear membrane disassembly [GO:0051078]; is part of meiosis II [GO:0007135] Definition: The controlled breakdown of the nuclear membranes during the second division of meiosis. Sources: GOC:bf Also known as: meiosis II nuclear envelope breakdown, meiosis II nuclear envelope catabolism, meiosis II nuclear envelope degradation, meiosis II nuclear envelope disassembly